{
  "term_id": "GO:0007283",
  "gene": "UniProtKB:Q9Y4R7",
  "gene_name": "Tubulin monoglycylase TTLL3",
  "gene_symbol": "TTLL3",
  "term_label": "spermatogenesis"
}